{
  "gene": "UniProtKB:Q8IV77",
  "term_label": "intracellularly cGMP-activated cation channel activity",
  "gene_symbol": "CNGA4",
  "gene_name": "Cyclic nucleotide-gated cation channel alpha-4",
  "term_id": "GO:0005223"
}